mammary gland branching involved in thelarche [GO:0060744] (biological process) Definition: The process in which the branching structure of the mammary gland duct is generated and organized during the period of sexual maturity in mammals. The mammary gland is a large compound sebaceous gland that in female mammals is modified to secrete milk. Relationships: is a type of GO:0060444; is part of thelarche [GO:0042695] References: PMID:19261859 Sources: GOC:dph Also known as: mammary gland branching involved in puberty